{
  "gene": "UniProtKB:O15270",
  "gene_symbol": "SPTLC2",
  "gene_name": "Serine palmitoyltransferase 2",
  "term_id": "GO:0046513",
  "term_label": "ceramide biosynthetic process"
}